type B pancreatic cell apoptotic process [GO:0097050] (BP) Definition: Any apoptotic process in a type B pancreatic cell, a cell located towards center of the islets of Langerhans that secretes insulin. References: PMID:16087305 Sources: CL:0000169, GOC:BHF, GOC:mtg_apoptosis Also known as: pancreatic B cell apoptosis, pancreatic beta cell apoptosis, type B pancreatic cell apoptosis Relationships: is a type of epithelial cell apoptotic process [GO:1904019] Regulation: RO_0002211 by regulation of type B pancreatic cell apoptotic process [GO:2000674]; negatively regulated by negative regulation of type B pancreatic cell apoptotic process [GO:2000675]; positively regulated by positive regulation of type B pancreatic cell apoptotic process [GO:2000676]